regulation of translational fidelity [GO:0006450] (biological process) Definition: Any process that modulates the ability of the translational apparatus to interpret the genetic code. Sources: GOC:dph, GOC:tb Also known as: regulation of translational accuracy Relationships: is a type of regulation of biological quality [GO:0065008] Subtypes: negative regulation of translational fidelity [GO:0045902], positive regulation of translational fidelity [GO:0045903], aminoacyl-tRNA metabolism involved in translational fidelity [GO:0106074], regulation of cytoplasmic translational fidelity [GO:0140018]